{
  "term_id": "GO:0004674",
  "gene": "UniProtKB:P0C264",
  "gene_name": "Uncharacterized serine_threonine-protein kinase SBK3",
  "gene_symbol": "SBK3",
  "term_label": "protein serine/threonine kinase activity"
}